{
  "gene_symbol": "ZNF157",
  "term_id": "UNKNOWN:0002",
  "term_label": "Unknown biological process",
  "gene": "UniProtKB:P51786",
  "gene_name": "Zinc finger protein 157"
}